cellular response to aldosterone [GO:1904045] (biological process) References: PMID:17644563 Sources: GOC:TermGenie, GO_REF:0000071 Definition: Any process that results in a change in state or activity of a cell (in terms of movement, secretion, enzyme production, gene expression, etc.) as a result of an aldosterone stimulus. Relationships: is a type of cellular response to mineralocorticoid stimulus [GO:0071389]; is a type of cellular response to alcohol [GO:0097306]; is a type of cellular response to aldehyde [GO:0110096]; is a type of GO:1901655; is a type of response to aldosterone [GO:1904044]